postsynaptic specialization organization [GO:0099084] (biological process) Subtypes: GO:0097106, postsynaptic specialization assembly [GO:0098698] Relationships: is a type of organelle organization [GO:0006996]; is part of postsynapse organization [GO:0099173] References: PMID:21525273, PMID:26834556 Sources: GOC:BHF, GOC:sjp Definition: A process that results in the assembly, arrangement of constituent parts, or disassembly of a postsynaptic specialization, a structure that lies adjacent to the cytoplasmic face of the postsynaptic membrane. Also known as: post synaptic specialization organization, post-synaptic specialization organization, postsynaptic specialization organisation